{
  "gene_name": "StAR-related lipid transfer protein 8",
  "gene_symbol": "STARD8",
  "term_label": "actin cytoskeleton organization",
  "gene": "UniProtKB:Q92502",
  "term_id": "GO:0030036"
}